{
  "term_id": "GO:0061631",
  "gene_symbol": "UBE2H",
  "gene_name": "Ubiquitin-conjugating enzyme E2 H",
  "term_label": "ubiquitin conjugating enzyme activity",
  "gene": "UniProtKB:P62256"
}